{
  "gene_symbol": "TMEM199",
  "term_id": "UNKNOWN:0002",
  "term_label": "Unknown biological process",
  "gene_name": "Transmembrane protein 199",
  "gene": "UniProtKB:Q8N511"
}